{
  "term_label": "plasma membrane",
  "term_id": "GO:0005886",
  "gene_name": "Roundabout homolog 3",
  "gene_symbol": "ROBO3",
  "gene": "UniProtKB:Q96MS0"
}